{
  "term_label": "ubiquitin conjugating enzyme activity",
  "gene": "UniProtKB:Q8WVN8",
  "term_id": "GO:0061631",
  "gene_name": "Ubiquitin-conjugating enzyme E2 Q2",
  "gene_symbol": "UBE2Q2"
}